{
  "gene": "UniProtKB:P01213",
  "gene_name": "Proenkephalin-B",
  "term_label": "axon terminus",
  "term_id": "GO:0043679",
  "gene_symbol": "PDYN"
}